growth hormone receptor activity [GO:0004903] (molecular function) Relationships: is a type of cytokine receptor activity [GO:0004896] Definition: Combining with a growth hormone and transmitting the signal from one side of the membrane to the other to initiate a change in cell activity. Sources: GOC:ai, GOC:signaling